homoserine transmembrane transporter activity [GO:0042970] (MF) Definition: Enables the transfer of homoserine from one side of a membrane to the other. Homoserine is alpha-amino-gamma-hydroxybutyric acid, an intermediate in the biosynthesis of cystathionine, threonine and methionine. Also known as: homoserine transporter activity Relationships: is a type of GO:0015175; is a type of GO:0015179; is part of GO:0042968 Sources: GOC:go_curators, ISBN:0198506732